{
  "gene_name": "Centrin-1",
  "term_id": "GO:0005509",
  "term_label": "calcium ion binding",
  "gene": "UniProtKB:Q12798",
  "gene_symbol": "CETN1"
}